{
  "term_label": "regulation of synaptic vesicle exocytosis",
  "gene_symbol": "RIMS3",
  "term_id": "GO:2000300",
  "gene": "UniProtKB:Q9UJD0",
  "gene_name": "Regulating synaptic membrane exocytosis protein 3"
}